{
  "gene_name": "AN1-type zinc finger protein 2A",
  "gene_symbol": "ZFAND2A",
  "term_label": "Unknown molecular function",
  "gene": "UniProtKB:Q8N6M9",
  "term_id": "UNKNOWN:0001"
}